{
  "gene_symbol": "FLT3",
  "term_label": "growth factor binding",
  "term_id": "GO:0019838",
  "gene": "UniProtKB:P36888",
  "gene_name": "Receptor-type tyrosine-protein kinase FLT3"
}